{
  "gene": "UniProtKB:Q12996",
  "term_label": "mRNA binding",
  "term_id": "GO:0003729",
  "gene_name": "Cleavage stimulation factor subunit 3",
  "gene_symbol": "CSTF3"
}